L-lyxose metabolic process [GO:0019324] (biological process) Sources: GOC:jsg, GOC:mah, ISBN:0198506732 Also known as: L-lyxose metabolism Definition: The chemical reactions and pathways involving L-lyxose, the L-enantiomer of aldopentose lyxo-pentose, the C-2 epimer of xylose. Relationships: is a type of GO:0019321